{
  "term_label": "angiotensin-activated signaling pathway",
  "term_id": "GO:0038166",
  "gene": "UniProtKB:P30556",
  "gene_name": "Type-1 angiotensin II receptor",
  "gene_symbol": "AGTR1"
}